{
  "gene": "UniProtKB:Q9BXS5",
  "gene_name": "AP-1 complex subunit mu-1",
  "term_label": "clathrin adaptor activity",
  "gene_symbol": "AP1M1",
  "term_id": "GO:0035615"
}